{
  "term_id": "GO:0017087",
  "gene": "UniProtKB:P31930",
  "gene_name": "Cytochrome b-c1 complex subunit 1, mitochondrial",
  "gene_symbol": "UQCRC1",
  "term_label": "mitochondrial processing peptidase complex"
}